cellular response to leukotriene B4 [GO:1905390] (biological process) References: PMID:14656734 Sources: GOC:TermGenie, GO_REF:0000071 Definition: Any process that results in a change in state or activity of a cell (in terms of movement, secretion, enzyme production, gene expression, etc.) as a result of a leukotriene B4 stimulus. Also known as: cellular response to LTB4 Relationships: is a type of GO:0071398; is a type of GO:1905389